{
  "gene_name": "Ubiquitin carboxyl-terminal hydrolase 7",
  "gene": "UniProtKB:Q93009",
  "term_id": "GO:0005829",
  "term_label": "cytosol",
  "gene_symbol": "USP7"
}